{
  "term_id": "GO:0005769",
  "gene_name": "Amyloid-beta precursor protein",
  "gene_symbol": "APP",
  "term_label": "early endosome",
  "gene": "UniProtKB:P05067"
}